{
  "term_label": "intermediate filament cytoskeleton organization",
  "term_id": "GO:0045104",
  "gene": "UniProtKB:Q03001",
  "gene_name": "Dystonin",
  "gene_symbol": "DST"
}